histone H3T3 kinase activity [GO:0072354] (molecular function) Definition: Catalysis of the reaction: histone H3-threonine (position 3) + ATP = histone H3-phosphothreonine (position 3) + ADP. This reaction is the addition of a phosphate group to the threonine residue at position 3 of histone H3. Note: Comment: Note that the residue position corresponds to the canonical human H3 histone (UniProtKB:P84243); this residue is conserved across all eukaryotes. Residue 1 is the first residue following removal of the initiating Methionine (Met). Note that each histone is encoded by multiple genes, and sequences may vary across different genes within an organism. Sources: GOC:mah Relationships: is a type of protein serine/threonine kinase activity [GO:0004674]; is a type of histone H3 kinase activity [GO:0140996] Also known as: histone H3-T3 kinase activity, histone kinase activity (H3-T3 specific), histone threonine kinase activity (H3-T3 specific), histone-threonine kinase activity (H3-T3 specific)